negative regulation of synaptic plasticity [GO:0031914] (biological process) Definition: A process that decreases synaptic plasticity, the ability of synapses to change as circumstances require. They may alter function, such as increasing or decreasing their sensitivity, or they may increase or decrease in actual numbers. Sources: GOC:mah Also known as: down regulation of synaptic plasticity, down-regulation of synaptic plasticity, downregulation of synaptic plasticity, inhibition of synaptic plasticity Relationships: is a type of regulation of synaptic plasticity [GO:0048167] Subtypes: negative regulation of synaptic metaplasticity [GO:0031917]